{
  "term_label": "RNA splicing",
  "term_id": "GO:0008380",
  "gene_symbol": "SMU1",
  "gene_name": "WD40 repeat-containing protein SMU1",
  "gene": "UniProtKB:Q2TAY7"
}